{
  "term_label": "mitochondrion",
  "term_id": "GO:0005739",
  "gene_name": "Cytochrome c oxidase assembly factor 8",
  "gene": "UniProtKB:Q96IL0",
  "gene_symbol": "COA8"
}